positive regulation of keratinocyte differentiation [GO:0045618] (biological process) Definition: Any process that activates or increases the frequency, rate or extent of keratinocyte differentiation. Also known as: up regulation of keratinocyte differentiation, up-regulation of keratinocyte differentiation, upregulation of keratinocyte differentiation, activation of keratinocyte differentiation, stimulation of keratinocyte differentiation Relationships: is_a positive regulation of epidermal cell differentiation [GO:0045606]; is a type of GO:0045616; is a type of positive regulation of multicellular organismal process [GO:0051240]; positively regulates keratinocyte differentiation [GO:0030216] Sources: GOC:go_curators